positive regulation of hemoglobin biosynthetic process [GO:0046985] (biological process) Definition: Any process that activates or increases the frequency, rate or extent of the chemical reactions and pathways resulting in the formation of hemoglobin, an oxygen carrying, conjugated protein containing four heme groups and globin. Sources: GOC:ai Also known as: positive regulation of haemoglobin biosynthesis, positive regulation of haemoglobin biosynthetic process, positive regulation of hemoglobin anabolism, positive regulation of hemoglobin biosynthesis, positive regulation of hemoglobin formation, positive regulation of hemoglobin synthesis, up regulation of hemoglobin biosynthetic process, up-regulation of hemoglobin biosynthetic process, upregulation of hemoglobin biosynthetic process, activation of hemoglobin biosynthetic process, stimulation of hemoglobin biosynthetic process Relationships: is a type of positive regulation of macromolecule biosynthetic process [GO:0010557]; is a type of regulation of hemoglobin biosynthetic process [GO:0046984]; is a type of positive regulation of protein metabolic process [GO:0051247]; positively regulates GO:0042541